meiotic drive [GO:0110134] (biological process) Relationships: is_a reproductive process [GO:0022414] Definition: A biological process that results in the unequal transmission of alleles, haplotypes, or chromosomes from a parental genome to gametes. In the absence of meiotic drive, the two copies of each gene or chromosome in a diploid organism are transmitted to offspring with equal probability, whereas meiotic drive results in overrepresentation of the driving allele among the surviving products of meiosis. References: PMID:26920473, PMID:29322557, PMID:29499907 Sources: GOC:mah